{
  "gene_name": "Killer cell immunoglobulin-like receptor, two Ig domains pseudogene 1",
  "term_label": "plasma membrane",
  "gene_symbol": "KIR2DP1",
  "term_id": "GO:0005886",
  "gene": "UniProtKB:A0A0G2JNF4"
}